{
  "term_id": "GO:0072345",
  "term_label": "NAADP-sensitive calcium-release channel activity",
  "gene": "UniProtKB:Q8IZK6",
  "gene_symbol": "MCOLN2",
  "gene_name": "Mucolipin-2"
}